{
  "term_label": "proton motive force-driven ATP synthesis",
  "gene_name": "ATP synthase subunit d, mitochondrial",
  "gene_symbol": "ATP5PD",
  "gene": "UniProtKB:O75947",
  "term_id": "GO:0015986"
}